{
  "term_label": "plasma membrane",
  "term_id": "GO:0005886",
  "gene": "UniProtKB:O43749",
  "gene_symbol": "OR1F1",
  "gene_name": "Olfactory receptor 1F1"
}